{
  "term_label": "Unknown biological process",
  "gene_name": "Cell growth regulator with EF hand domain protein 1",
  "gene": "UniProtKB:Q99674",
  "gene_symbol": "CGREF1",
  "term_id": "UNKNOWN:0002"
}